{
  "term_id": "GO:0032007",
  "term_label": "negative regulation of TOR signaling",
  "gene_name": "Tuberin",
  "gene_symbol": "TSC2",
  "gene": "UniProtKB:P49815"
}